{
  "gene_symbol": "RAB27A",
  "gene": "UniProtKB:P51159",
  "term_id": "GO:0045921",
  "gene_name": "Ras-related protein Rab-27A",
  "term_label": "positive regulation of exocytosis"
}